{
  "gene": "UniProtKB:Q9H5Q4",
  "term_label": "mitochondrial matrix",
  "gene_name": "Dimethyladenosine transferase 2, mitochondrial",
  "gene_symbol": "TFB2M",
  "term_id": "GO:0005759"
}